{
  "gene": "UniProtKB:Q9BZ95",
  "term_label": "chromatin",
  "gene_symbol": "NSD3",
  "term_id": "GO:0000785",
  "gene_name": "Histone-lysine N-methyltransferase NSD3"
}